{
  "gene_symbol": "TNIP2",
  "term_label": "positive regulation of canonical NF-kappaB signal transduction",
  "gene_name": "TNFAIP3-interacting protein 2",
  "gene": "UniProtKB:Q8NFZ5",
  "term_id": "GO:0043123"
}